negative regulation of natural killer cell mediated cytotoxicity directed against tumor cell target [GO:0002859] (biological process) Definition: Any process that stops, prevents, or reduces the frequency, rate, or extent of natural killer cell mediated cytotoxicity directed against tumor cell target. Sources: GOC:add Also known as: down regulation of natural killer cell mediated cytotoxicity directed against tumor cell target, down-regulation of natural killer cell mediated cytotoxicity directed against tumor cell target, downregulation of natural killer cell mediated cytotoxicity directed against tumor cell target, inhibition of natural killer cell mediated cytotoxicity directed against tumor cell target Relationships: is a type of negative regulation of natural killer cell mediated immune response to tumor cell [GO:0002856]; is a type of regulation of natural killer cell mediated cytotoxicity directed against tumor cell target [GO:0002858]; is a type of negative regulation of natural killer cell mediated cytotoxicity [GO:0045953]; negatively regulates natural killer cell mediated cytotoxicity directed against tumor cell target [GO:0002420]